chromosome condensation [GO:0030261] (biological process) Also known as: DNA condensation, eukaryotic chromosome condensation, nuclear chromosome condensation Subtypes: mitotic chromosome condensation [GO:0007076], GO:0010032, GO:0030263, rDNA chromatin condensation [GO:0070550] Sources: GOC:mah, ISBN:0815316194 Relationships: is a type of chromosome organization [GO:0051276] Regulation: regulated by GO:0060623; negatively regulated by negative regulation of chromosome condensation [GO:1902340]; positively regulated by GO:1905821 Definition: The progressive compaction of dispersed interphase chromatin into threadlike chromosomes prior to mitotic or meiotic nuclear division, or during apoptosis, in eukaryotic cells.